xenobiotic detoxification by transmembrane export across the plasma membrane [GO:1990961] (biological process) Regulation: regulated by GO:1905699; negatively regulated by negative regulation of xenobiotic detoxification by transmembrane export across the plasma membrane [GO:1905700]; positively regulated by positive regulation of xenobiotic detoxification by transmembrane export across the plasma membrane [GO:1905701] Relationships: is a type of xenobiotic export from cell [GO:0046618]; is a type of GO:0140115; is part of GO:0098754 Definition: A process that reduces or removes the toxicity of a xenobiotic by exporting it outside the cell. References: PMID:28355133 Also known as: drug transmembrane export